SUMO-ubiquitin ligase activity [GO:0140082] (MF) References: PMID:28552615 Definition: Isoenergetic transfer of SUMO from one protein to an existing ubiquitin chain via the reaction X-ubiquitin + Y-ubiquitin = Y-ubiquitin-ubiquitin + X, where both the X-ubiquitin and Y-ubiquitin-ubiquitin linkages are thioester bonds between the C-terminal glycine of ubiquitin and a sulfhydryl side group of a cysteine residue. Relationships: is a type of GO:0061665